{
  "gene_name": "Cyclic AMP-responsive element-binding protein 3-like protein 3",
  "gene": "UniProtKB:Q68CJ9",
  "term_label": "RNA polymerase II cis-regulatory region sequence-specific DNA binding",
  "gene_symbol": "CREB3L3",
  "term_id": "GO:0000978"
}